{
  "gene_name": "Striatin",
  "term_id": "GO:0016055",
  "gene_symbol": "STRN",
  "term_label": "Wnt signaling pathway",
  "gene": "UniProtKB:O43815"
}